{
  "term_id": "GO:2000304",
  "gene_name": "85_88 kDa calcium-independent phospholipase A2",
  "gene_symbol": "PLA2G6",
  "gene": "UniProtKB:O60733",
  "term_label": "positive regulation of ceramide biosynthetic process"
}